{
  "term_label": "microtubule severing ATPase activity",
  "term_id": "GO:0008568",
  "gene": "UniProtKB:Q5HY92",
  "gene_symbol": "FIGN",
  "gene_name": "Fidgetin"
}